regulation of ketone metabolic process [GO:0010565] (biological process) Subtypes: regulation of ecdysteroid metabolic process [GO:0007553], regulation of isopentenyl diphosphate biosynthetic process, methylerythritol 4-phosphate pathway [GO:0010322], regulation of salicylic acid metabolic process [GO:0010337], regulation of gibberellin biosynthetic process [GO:0010371], regulation of ketone biosynthetic process [GO:0010566], regulation of ketone catabolic process [GO:0010567], regulation of fatty acid metabolic process [GO:0019217], GO:0032344, regulation of acetate catabolic process [GO:0045734], regulation of bile acid biosynthetic process [GO:0070857], regulation of retinoic acid biosynthetic process [GO:1900052], regulation of methane biosynthetic process from formic acid [GO:1900339], regulation of fumonisin biosynthetic process [GO:1900683], regulation of gerfelin biosynthetic process [GO:1900686], regulation of o-orsellinic acid biosynthetic process [GO:1900698], regulation of ferulate catabolic process [GO:1901466], regulation of L-ascorbic acid biosynthetic process [GO:2000082], regulation of glyoxylate cycle [GO:2000874] Definition: Any process that modulates the chemical reactions and pathways involving any of a class of organic compounds that contain the carbonyl group, CO, and in which the carbonyl group is bonded only to carbon atoms. The general formula for a ketone is RCOR, where R and R are alkyl or aryl groups. Relationships: is_a regulation of metabolic process [GO:0019222]; regulates GO:0042180 Sources: GOC:dph, GOC:tb